{
  "gene": "UniProtKB:Q6ZSA8",
  "gene_symbol": "Q6ZSA8",
  "term_label": "Unknown biological process",
  "gene_name": "Putative uncharacterized protein FLJ45684",
  "term_id": "UNKNOWN:0002"
}